receptor metabolic process [GO:0043112] (biological process) Also known as: receptor metabolism Sources: GOC:jl Subtypes: receptor recycling [GO:0001881], low-density lipoprotein receptor particle metabolic process [GO:0032799], receptor catabolic process [GO:0032801] Relationships: is a type of macromolecule metabolic process [GO:0043170] Definition: The chemical reactions and pathways involving a receptor molecule, a macromolecule that undergoes combination with a hormone, neurotransmitter, drug or intracellular messenger to initiate a change in cell function.